motor behavior [GO:0061744] (biological process) Relationships: is a type of behavior [GO:0007610] Definition: The specific neuromuscular movement of a single organism in response to external or internal stimuli. Subtypes: psychomotor behavior [GO:0036343] References: PMID:25318560 Sources: GOC:PARL, GOC:bf